{
  "gene_symbol": "CYP2R1",
  "term_id": "GO:0042359",
  "term_label": "vitamin D metabolic process",
  "gene": "UniProtKB:Q6VVX0",
  "gene_name": "Vitamin D 25-hydroxylase"
}